CGG codon-amino acid adaptor activity [GO:0033432] (molecular function) Sources: GOC:mah Relationships: is a type of triplet codon-amino acid adaptor activity [GO:0030533] Note: Note that in the standard genetic code, CGG codes for arginine. Definition: A triplet codon-amino acid adaptor activity that recognizes a CGG codon. Also known as: arginine tRNA